{
  "gene": "UniProtKB:Q9BRF8",
  "term_label": "Unknown cellular component",
  "gene_name": "Serine_threonine-protein phosphatase CPPED1",
  "term_id": "UNKNOWN:0003",
  "gene_symbol": "CPPED1"
}